eye-antennal disc development [GO:0035214] (biological process) Relationships: is_a imaginal disc development [GO:0007444] Sources: GOC:bf, ISBN:0879694238 Definition: Progression of the eye-antennal imaginal disc over time, from its initial formation through to its metamorphosis to form adult structures including the eye, antenna, head capsule and maxillary palps.